{
  "gene": "UniProtKB:Q6UWF9",
  "term_label": "Unknown cellular component",
  "term_id": "UNKNOWN:0003",
  "gene_symbol": "FAM180A",
  "gene_name": "Protein FAM180A"
}